RNA polymerase V transcription repressor complex [GO:0090574] (cellular component) Sources: GOC:tb Definition: A protein complex, located in the nucleus, that possesses activity that prevents or downregulates transcription from a RNA polymerase V promoter. Relationships: is a type of transcription repressor complex [GO:0017053]; is a type of nuclear protein-containing complex [GO:0140513]